{
  "term_label": "positive regulation of pseudopodium assembly",
  "gene": "UniProtKB:O14613",
  "term_id": "GO:0031274",
  "gene_symbol": "CDC42EP2",
  "gene_name": "Cdc42 effector protein 2"
}